steviolbioside glucosyltransferase activity (rebaudioside B forming) [GO:0102380] (molecular function) Relationships: is a type of GO:0016758 Definition: Catalysis of the reaction: steviolbioside + UDP-alpha-D-glucose = H+ + rebaudioside B + UDP. Sources: RHEA:61752